{
  "gene_name": "DNA helicase B",
  "gene_symbol": "HELB",
  "term_label": "DNA-templated DNA replication",
  "gene": "UniProtKB:Q8NG08",
  "term_id": "GO:0006261"
}